{
  "gene": "UniProtKB:Q9Y678",
  "gene_symbol": "COPG1",
  "term_id": "GO:0030126",
  "term_label": "COPI vesicle coat",
  "gene_name": "Coatomer subunit gamma-1"
}